{
  "gene_name": "Ubiquitin-conjugating enzyme E2 D4",
  "term_label": "ubiquitin conjugating enzyme activity",
  "term_id": "GO:0061631",
  "gene": "UniProtKB:Q9Y2X8",
  "gene_symbol": "UBE2D4"
}